ureter morphogenesis [GO:0072197] (BP) Definition: The process in which the anatomical structures of the ureter are generated and organized. The ureter is a muscular tube that transports urine from the kidney to the urinary bladder. Sources: GOC:mtg_kidney_jan10 Relationships: is a type of animal organ morphogenesis [GO:0009887]; is a type of tube morphogenesis [GO:0035239]; is part of GO:0072189